{
  "term_id": "GO:0043484",
  "gene_symbol": "RBM20",
  "gene_name": "RNA-binding protein 20",
  "gene": "UniProtKB:Q5T481",
  "term_label": "regulation of RNA splicing"
}